{
  "term_id": "GO:0016887",
  "term_label": "ATP hydrolysis activity",
  "gene_symbol": "AFG1L",
  "gene_name": "AFG1-like ATPase",
  "gene": "UniProtKB:Q8WV93"
}